{
  "term_label": "eye development",
  "gene_symbol": "MEIS1",
  "term_id": "GO:0001654",
  "gene": "UniProtKB:O00470",
  "gene_name": "Homeobox protein Meis1"
}